{
  "gene_symbol": "RUSC2",
  "gene": "UniProtKB:Q8N2Y8",
  "term_label": "Unknown molecular function",
  "term_id": "UNKNOWN:0001",
  "gene_name": "AP-4 complex accessory subunit RUSC2"
}